{
  "gene_name": "Zinc finger protein 684",
  "term_id": "GO:0005634",
  "gene_symbol": "ZNF684",
  "term_label": "nucleus",
  "gene": "UniProtKB:Q5T5D7"
}